{
  "gene": "UniProtKB:Q15058",
  "term_label": "microtubule-based movement",
  "term_id": "GO:0007018",
  "gene_name": "Kinesin-like protein KIF14",
  "gene_symbol": "KIF14"
}